{
  "term_label": "Unknown molecular function",
  "term_id": "UNKNOWN:0001",
  "gene_name": "Transmembrane protein 151A",
  "gene_symbol": "TMEM151A",
  "gene": "UniProtKB:Q8N4L1"
}